siderophore-iron transmembrane transporter activity [GO:0015343] (molecular function) Relationships: is a type of iron chelate transmembrane transporter activity [GO:0015603] Definition: Enables the transfer of a solute or solutes from one side of a membrane to the other according to the reaction: siderophore-iron(out) + H+(out) = siderophore-iron(in) + H+(in). References: PMID:20376388, PMID:31748738 Subtypes: siderophore uptake transmembrane transporter activity [GO:0015344], ferric triacetylfusarinine C:proton symporter activity [GO:0015346], GO:0015620, ferrichrome transmembrane transporter activity [GO:0042929], GO:0042931, GO:0042933, achromobactin transmembrane transporter activity [GO:0042934] Also known as: iron-siderophore transporter activity, siderochrome transporter activity, siderochrome-iron transporter activity, siderophore transmembrane transporter activity, siderophore transporter activity, siderophore-iron transporter activity